{
  "gene": "UniProtKB:Q08357",
  "term_id": "GO:0005315",
  "gene_symbol": "SLC20A2",
  "gene_name": "Sodium-dependent phosphate transporter 2",
  "term_label": "phosphate transmembrane transporter activity"
}